histone H3K27cr reader activity [GO:0140038] (molecular function) Definition: A histone reader that recognizes a histone H3 crotonylated at lysine 27. Also known as: histone H3K27cr modified histone binding Relationships: is a type of histone H3 reader activity [GO:0140006] Note: Comment: Note that the residue position corresponds to the canonical human H3 histone (UniProtKB:P84243); this residue is conserved across all eukaryotes. Residue 1 is the first residue following removal of the initiating Methionine (Met). Note that each histone is encoded by multiple genes, and sequences may vary across different genes within an organism. References: PMID:27105114